intramolecular hydroxytransferase activity [GO:0050486] (molecular function) Subtypes: isochorismate synthase activity [GO:0008909], GO:0018824, 3-(hydroxyamino)phenol mutase activity [GO:0034022], 9,12-octadecadienoate 8-hydroperoxide 8S-isomerase activity [GO:0052879], hydroperoxy icosatetraenoate isomerase activity [GO:0106255] Definition: Catalysis of the transfer of a hydroxyl group from one position to another within a single molecule. Relationships: is a type of intramolecular transferase activity [GO:0016866] Also known as: intramolecular transferase activity, transferring hydroxy groups Sources: GOC:mah